{
  "term_label": "retinal metabolic process",
  "gene_symbol": "DHRS4L1",
  "gene_name": "Putative dehydrogenase_reductase SDR family member 4-like 1",
  "term_id": "GO:0042574",
  "gene": "UniProtKB:P0CG22"
}